{
  "term_label": "integrin binding",
  "gene_name": "Semaphorin-7A",
  "term_id": "GO:0005178",
  "gene": "UniProtKB:O75326",
  "gene_symbol": "SEMA7A"
}